{
  "term_id": "UNKNOWN:0003",
  "gene_name": "Delphilin",
  "gene": "UniProtKB:A4D2P6",
  "term_label": "Unknown cellular component",
  "gene_symbol": "GRID2IP"
}